{
  "term_id": "GO:0005509",
  "gene_name": "Sorcin",
  "term_label": "calcium ion binding",
  "gene_symbol": "SRI",
  "gene": "UniProtKB:P30626"
}